venom-mediated fibrinolysis [GO:0044484] (biological process) References: PMID:17433397, PMID:17544404 Sources: GOC:fj, GOC:jl Also known as: envenomation resulting in fibrinolysis, envenomation resulting in fibrinolysis in another organism, envenomation resulting in fibrinolysis in other organism Subtypes: venom-mediated plasminogen activation [GO:0044544] Relationships: is a type of venom-mediated perturbation of hemostasis [GO:0044483] Definition: A process in which an organism causes fibrinolysis in another organism via the action of a venom. Fibrinolysis is a process that solubilizes fibrin in the blood, chiefly by the proteolytic action of plasmin.